{
  "gene_name": "ADP-ribosylation factor-like protein 6",
  "gene_symbol": "ARL6",
  "gene": "UniProtKB:Q9H0F7",
  "term_label": "intracellular protein transport",
  "term_id": "GO:0006886"
}